{
  "gene_name": "T cell receptor beta variable 6-4",
  "gene": "UniProtKB:A0A1B0GX49",
  "gene_symbol": "TRBV6-4",
  "term_id": "GO:0007166",
  "term_label": "cell surface receptor signaling pathway"
}